{
  "gene": "UniProtKB:Q8WVP5",
  "gene_name": "Tumor necrosis factor alpha-induced protein 8-like protein 1",
  "gene_symbol": "TNFAIP8L1",
  "term_label": "cytoplasm",
  "term_id": "GO:0005737"
}